{
  "term_id": "UNKNOWN:0001",
  "gene": "UniProtKB:Q8TAA9",
  "term_label": "Unknown molecular function",
  "gene_name": "Vang-like protein 1",
  "gene_symbol": "VANGL1"
}